shell calcification [GO:0031215] (biological process) Definition: The precipitation of calcium carbonate onto the organic matrix of a shell, such as a mollusc shell. Relationships: is a type of biomineral tissue development [GO:0031214] Regulation: regulated by regulation of shell calcification [GO:1905648]; RO_0002212 by GO:1905649; positively regulated by positive regulation of shell calcification [GO:1905650] References: PMID:15132736 Sources: GOC:mah